{
  "gene_name": "Maestro heat-like repeat-containing protein family member 6",
  "gene": "UniProtKB:A6NGR9",
  "gene_symbol": "MROH6",
  "term_id": "UNKNOWN:0001",
  "term_label": "Unknown molecular function"
}